{
  "gene_name": "Thioredoxin domain-containing protein 12",
  "term_label": "Unknown molecular function",
  "gene_symbol": "TXNDC12",
  "term_id": "UNKNOWN:0001",
  "gene": "UniProtKB:O95881"
}